{
  "gene_symbol": "RNLS",
  "gene_name": "Renalase",
  "term_id": "GO:0005576",
  "term_label": "extracellular region",
  "gene": "UniProtKB:Q5VYX0"
}